larval walking behavior [GO:0008346] (biological process) Sources: GOC:go_curators, GOC:pr Definition: The behavior of a larval organism relating to the progression of that organism along the ground by the process of lifting and setting down each leg. Relationships: is a type of larval locomotory behavior [GO:0008345]; is a type of walking behavior [GO:0090659] Also known as: larval walking behaviour